{
  "term_label": "SUMO activating enzyme complex",
  "gene": "UniProtKB:Q9UBE0",
  "term_id": "GO:0031510",
  "gene_symbol": "SAE1",
  "gene_name": "SUMO-activating enzyme subunit 1"
}